{
  "gene_symbol": "THOC7",
  "term_id": "GO:0006406",
  "gene": "UniProtKB:Q6I9Y2",
  "gene_name": "THO complex subunit 7 homolog",
  "term_label": "mRNA export from nucleus"
}